collagen type XIX trimer [GO:1990318] (cellular component) References: PMID:10585282, PMID:12579531, PMID:12788917, PMID:17876790, PMID:31823868, PMID:35346795, PMID:9403723 Relationships: is a type of collagen trimer [GO:0005581]; is part of collagenous component of basement membrane [GO:0140143] Note: The collagen XIX trimer is often classified as a FACIT collagen trimer (which stands for Fibril Associated Collagens with Interrupted Triple helices) because of the presence of interrupted triple helical collagen domains, similar to other FACIT members. However, evidence show that collagen XIX localizes to basement membrane ECMs, and none of the basement membrane collagens are fibrillar. Definition: A collagen homotrimer made of three alpha1(XIX) collagen chains, each presenting interrupted triple helical collagen domains. Localizes to basement membrane ECMs, not known to associate with any fibrillar collagens that are predominantly found in the interstitial extracellular matrix.